{
  "term_label": "synapse",
  "term_id": "GO:0045202",
  "gene_symbol": "POTEE",
  "gene": "UniProtKB:Q6S8J3",
  "gene_name": "POTE ankyrin domain family member E"
}